Toll-like receptor 2-Toll-like receptor 6 protein complex [GO:0035355] (cellular component) Relationships: is a type of GO:0098802 References: PMID:19931471, PMID:21481769 Sources: GOC:add, GOC:signaling Also known as: TLR2-TLR6 protein complex, TLR2:TLR6 heterodimer, TLR6:TLR2 complex, toll-like receptor TLR6:TLR2 heterodimeric complex Definition: A heterodimeric protein complex containing Toll-like receptor 2 (TLR2) and Toll-like receptor 6 (TLR6).